{
  "gene_name": "Cytochrome P450 4F2",
  "gene_symbol": "CYP4F2",
  "gene": "UniProtKB:P78329",
  "term_label": "Unknown cellular component",
  "term_id": "UNKNOWN:0003"
}